regulation of Arp2/3 complex-mediated actin nucleation [GO:0034315] (biological process) Definition: Any process that modulates the frequency, rate or extent of actin nucleation mediated by the Arp2/3 complex and interacting proteins. Relationships: is a type of GO:0051125; regulates Arp2/3 complex-mediated actin nucleation [GO:0034314] Subtypes: negative regulation of Arp2/3 complex-mediated actin nucleation [GO:0034316], positive regulation of Arp2/3 complex-mediated actin nucleation [GO:2000601] Sources: GOC:mah